{
  "term_label": "insulin-like growth factor II binding",
  "gene": "UniProtKB:P22692",
  "gene_symbol": "IGFBP4",
  "gene_name": "Insulin-like growth factor-binding protein 4",
  "term_id": "GO:0031995"
}